{
  "term_label": "flavone metabolic process",
  "term_id": "GO:0051552",
  "gene_name": "UDP-glucuronosyltransferase 1A9",
  "gene": "UniProtKB:O60656",
  "gene_symbol": "UGT1A9"
}